fatty-acyl-CoA synthase complex [GO:0005836] (cellular component) Definition: A protein complex that possesses fatty-acyl-CoA synthase activity. Note: Note that fatty acid synthetases of vertebrates and yeast are stable enzyme complexes of multifunctional polypeptide chains, whereas the fatty acid synthetases of plants and E. coli consist of non-associated individual enzymes. Relationships: is a type of transferase complex [GO:1990234]; is part of GO:0005829 Also known as: fatty acyl CoA synthase complex Sources: GOC:mah